{
  "term_label": "positive regulation of apoptotic process",
  "gene_symbol": "TNFRSF10A",
  "gene": "UniProtKB:O00220",
  "term_id": "GO:0043065",
  "gene_name": "Tumor necrosis factor receptor superfamily member 10A"
}